low-affinity IgE receptor activity [GO:0019769] (molecular function) Sources: GOC:add, GOC:signaling, ISBN:0781735149 Also known as: low affinity IgE receptor activity, low affinity Fc receptor activity Definition: Combining with low affinity with an immunoglobulin of the IgE isotype via the Fc region, and transmitting the signal from one side of the membrane to the other to initiate a change in cell activity. Relationships: is a type of IgE receptor activity [GO:0019767]